{
  "term_id": "GO:0001227",
  "gene_name": "Zinc finger and BTB domain-containing protein 14",
  "term_label": "DNA-binding transcription repressor activity, RNA polymerase II-specific",
  "gene": "UniProtKB:O43829",
  "gene_symbol": "ZBTB14"
}